cell-matrix recognition [GO:0009989] (biological process) Sources: ISBN:0824072820 Definition: Cell recognition that involves the interaction of the cell with the extracellular matrix. Subtypes: contact guidance [GO:0009990] Relationships: is a type of cell recognition [GO:0008037]